{
  "term_id": "UNKNOWN:0001",
  "gene": "UniProtKB:Q8N998",
  "gene_name": "Coiled-coil domain-containing protein 89",
  "term_label": "Unknown molecular function",
  "gene_symbol": "CCDC89"
}